{
  "gene_name": "FIGNL1-interacting regulator of recombination and mitosis",
  "term_label": "Unknown cellular component",
  "gene": "UniProtKB:Q9NSG2",
  "gene_symbol": "FIRRM",
  "term_id": "UNKNOWN:0003"
}